{
  "term_label": "substance P receptor activity",
  "term_id": "GO:0016496",
  "gene_symbol": "TACR1",
  "gene_name": "Substance-P receptor",
  "gene": "UniProtKB:P25103"
}